fusarinine-C ornithinesterase activity [GO:0047908] (molecular function) Relationships: is a type of GO:0052689 Also known as: 5-N-acyl-L-ornithine-ester hydrolase activity, N5-acyl-L-ornithine-ester hydrolase activity, ornithine esterase activity Definition: Catalysis of the reaction: N5-acyl-L-ornithine ester + H2O = N5-acyl-L-ornithine + an alcohol. Sources: EC:3.1.1.48, MetaCyc:FUSARININE-C-ORNITHINESTERASE-RXN